establishment of planar polarity involved in metanephric nephron morphogenesis [GO:0072280] (BP) Definition: Coordinated organization of groups of cells in the plane of an epithelium that contributes to the shaping of a nephron in the metanephros. Sources: GOC:mtg_kidney_jan10 Also known as: establishment of planar cell polarity involved in metanephric nephron morphogenesis Relationships: is a type of establishment of planar polarity involved in nephron morphogenesis [GO:0072046]; is part of metanephric nephron morphogenesis [GO:0072273]